{
  "gene": "UniProtKB:Q6RI45",
  "term_label": "Unknown molecular function",
  "gene_name": "Bromodomain and WD repeat-containing protein 3",
  "term_id": "UNKNOWN:0001",
  "gene_symbol": "BRWD3"
}